box C/D snoRNP assembly [GO:0000492] (biological process) Sources: GOC:krc Definition: The aggregation, arrangement and bonding together of proteins and a box C/D snoRNA to form a box C/D small nucleolar ribonucleoprotein (snoRNP) complex. Relationships: is a type of small nucleolar ribonucleoprotein complex assembly [GO:0000491] Also known as: box C/D small nucleolar ribonucleoprotein complex assembly